{
  "gene_symbol": "NKIRAS2",
  "term_label": "Ral protein signal transduction",
  "gene": "UniProtKB:Q9NYR9",
  "gene_name": "NF-kappa-B inhibitor-interacting Ras-like protein 2",
  "term_id": "GO:0032484"
}